{
  "gene": "UniProtKB:Q9BZK3",
  "term_label": "protein targeting to membrane",
  "gene_symbol": "NACA4P",
  "gene_name": "Putative nascent polypeptide-associated complex subunit alpha-like protein",
  "term_id": "GO:0006612"
}